{
  "gene_name": "Zinc finger protein Helios",
  "gene_symbol": "IKZF2",
  "gene": "UniProtKB:Q9UKS7",
  "term_id": "GO:0006357",
  "term_label": "regulation of transcription by RNA polymerase II"
}